{
  "gene_name": "Thioredoxin reductase 3",
  "gene_symbol": "TXNRD3",
  "term_label": "cell redox homeostasis",
  "term_id": "GO:0045454",
  "gene": "UniProtKB:Q86VQ6"
}